{
  "term_label": "structural constituent of cytoskeleton",
  "gene": "UniProtKB:Q9NY65",
  "gene_name": "Tubulin alpha-8 chain",
  "gene_symbol": "TUBA8",
  "term_id": "GO:0005200"
}